{
  "term_id": "GO:0042043",
  "gene": "UniProtKB:Q4VX76",
  "term_label": "neurexin family protein binding",
  "gene_name": "Synaptotagmin-like protein 3",
  "gene_symbol": "SYTL3"
}